{
  "term_id": "GO:0005768",
  "gene_symbol": "PTPN23",
  "gene_name": "Tyrosine-protein phosphatase non-receptor type 23",
  "term_label": "endosome",
  "gene": "UniProtKB:Q9H3S7"
}